{
  "gene": "UniProtKB:P33778",
  "term_label": "chromatin organization",
  "term_id": "GO:0006325",
  "gene_name": "Histone H2B type 1-B",
  "gene_symbol": "H2BC3"
}